{
  "gene": "UniProtKB:Q17RB8",
  "gene_symbol": "LONRF1",
  "gene_name": "LON peptidase N-terminal domain and RING finger protein 1",
  "term_id": "GO:0061630",
  "term_label": "ubiquitin protein ligase activity"
}